BIM-BCL-xl complex [GO:0097140] (CC) Definition: A heterodimeric protein complex consisting of BIM and BCL-xl, members of the Bcl-2 family of anti- and proapoptotic regulators. Relationships: is a type of Bcl-2 family protein complex [GO:0097136] References: PMID:14634621 Sources: GOC:so